{
  "term_id": "GO:0005047",
  "gene": "UniProtKB:Q9GZP9",
  "term_label": "signal recognition particle binding",
  "gene_name": "Derlin-2",
  "gene_symbol": "DERL2"
}